{
  "term_id": "GO:0007266",
  "term_label": "Rho protein signal transduction",
  "gene_symbol": "RACGAP1",
  "gene_name": "Rac GTPase-activating protein 1",
  "gene": "UniProtKB:Q9H0H5"
}